{
  "gene": "UniProtKB:Q0VDD8",
  "gene_symbol": "DNAH14",
  "term_label": "cilium movement involved in cell motility",
  "term_id": "GO:0060294",
  "gene_name": "Dynein axonemal heavy chain 14"
}